{
  "gene_symbol": "SLC36A2",
  "term_label": "L-alanine transport",
  "gene_name": "Proton-coupled amino acid transporter 2",
  "gene": "UniProtKB:Q495M3",
  "term_id": "GO:0015808"
}